eukaryotic 48S preinitiation complex [GO:0033290] (cellular component) Definition: The protein-ribosome-tRNA complex that has just recognized the start codon of a capped mRNA. It is composed of the small ribosomal subunit, eukaryote initiation factors (eIF) eIF3 complex, eIF1, eIF1A, eIF2-GDP, eIF4 complex and initiatior-methionine-tRNA. Recognition of the start codon triggers downstream steps in the pathway, including eIF1 dissociation; Pi release from eIF2; and conversion to the closed, scanning-arrested conformation of the PIC. References: PMID:16510876, PMID:24319994, PMID:24499181, PMID:29735639 Sources: GOC:hjd Also known as: eukaryotic 48S pre-initiation complex, eukaryotic 48S initiation complex Relationships: is a type of GO:0070993; has part cytosolic small ribosomal subunit [GO:0022627]